multivesicular body organization [GO:0036257] (biological process) Relationships: is a type of endosome organization [GO:0007032] Also known as: MVB organization Subtypes: multivesicular body assembly [GO:0036258] Definition: A process that is carried out at the cellular level which results in the assembly, arrangement of constituent parts, or disassembly of a multivesicular body. A multivesicular body is a type of late endosome in which regions of the limiting endosomal membrane invaginate to form internal vesicles; membrane proteins that enter the internal vesicles are sequestered from the cytoplasm. References: PMID:11566881 Sources: GOC:sart